3-hydroxyphenylpropionic acid transmembrane transport [GO:0042920] (biological process) Relationships: is a type of monocarboxylic acid transport [GO:0015718]; is a type of organic hydroxy compound transport [GO:0015850] References: PMID:9098055 Sources: GOC:go_curators Definition: The directed movement of 3-hydroxyphenylpropionic acid across a lipid bilayer, from one side of a membrane to the other. Also known as: 3-hydroxyphenylpropionic acid transport, 3-(3-hydroxyphenyl)propionic acid transport, m-hydroxyphenylpropionic acid transport